{
  "term_id": "GO:0022841",
  "gene": "UniProtKB:Q9Y2U2",
  "term_label": "potassium ion leak channel activity",
  "gene_name": "Potassium channel subfamily K member 7",
  "gene_symbol": "KCNK7"
}